{
  "gene": "UniProtKB:A0A0G2JMI3",
  "term_label": "antigen binding",
  "gene_name": "Immunoglobulin heavy variable 1-69-2",
  "term_id": "GO:0003823",
  "gene_symbol": "IGHV1-69-2"
}